{
  "term_label": "phospholipase C-activating G protein-coupled receptor signaling pathway",
  "term_id": "GO:0007200",
  "gene": "UniProtKB:Q9HB89",
  "gene_name": "Neuromedin-U receptor 1",
  "gene_symbol": "NMUR1"
}